{
  "gene_name": "Replication protein A 70 kDa DNA-binding subunit",
  "gene": "UniProtKB:P27694",
  "term_id": "GO:0005662",
  "term_label": "DNA replication factor A complex",
  "gene_symbol": "RPA1"
}